{
  "term_label": "SCF ubiquitin ligase complex",
  "term_id": "GO:0019005",
  "gene_symbol": "FBXL6",
  "gene_name": "F-box_LRR-repeat protein 6",
  "gene": "UniProtKB:Q8N531"
}